{
  "gene": "UniProtKB:Q9NZW4",
  "term_id": "GO:0005518",
  "gene_name": "Dentin sialophosphoprotein",
  "gene_symbol": "DSPP",
  "term_label": "collagen binding"
}